multivesicular body fusion to apical plasma membrane [GO:0098866] (biological process) Definition: The fusion of the membrane of a multivesicular body with the apical plasma membrane, resulting in release of exosomes from the cell. References: PMID:26459596 Relationships: is a type of vesicle fusion to plasma membrane [GO:0099500]; BFO_0000050 exosomal secretion [GO:1990182]